{
  "gene": "UniProtKB:O14787",
  "gene_symbol": "TNPO2",
  "gene_name": "Transportin-2",
  "term_label": "nuclear import signal receptor activity",
  "term_id": "GO:0061608"
}